spinal cord association neuron specification [GO:0021519] (biological process) Relationships: is a type of neuron fate specification [GO:0048665]; BFO_0000050 spinal cord association neuron differentiation [GO:0021527] Definition: The process in which a cell becomes capable of differentiating autonomously into an association neuron in an environment that is neutral with respect to the developmental pathway. Sources: GOC:cls, GOC:dgh, GOC:dph, GOC:jid, GO_REF:0000021